{
  "term_label": "sucrose:proton symporter activity",
  "term_id": "GO:0008506",
  "gene": "UniProtKB:Q5BKX6",
  "gene_symbol": "SLC45A4",
  "gene_name": "Solute carrier family 45 member 4"
}